{
  "term_label": "immunoglobulin complex",
  "gene": "UniProtKB:A0A1B0GX56",
  "term_id": "GO:0019814",
  "gene_symbol": "TRDV1",
  "gene_name": "T cell receptor delta variable 1"
}